{
  "gene_symbol": "FGF8",
  "term_label": "positive regulation of MAPK cascade",
  "gene_name": "Fibroblast growth factor 8",
  "gene": "UniProtKB:P55075",
  "term_id": "GO:0043410"
}